{
  "term_id": "UNKNOWN:0002",
  "term_label": "Unknown biological process",
  "gene": "UniProtKB:Q9BYQ2",
  "gene_symbol": "KRTAP9-4",
  "gene_name": "Keratin-associated protein 9-4"
}